{
  "term_id": "UNKNOWN:0002",
  "gene_symbol": "A0A7I2V2S6",
  "gene": "UniProtKB:A0A7I2V2S6",
  "term_label": "Unknown biological process",
  "gene_name": "Uncharacterized protein"
}